regulation of synaptic vesicle clustering [GO:2000807] (biological process) Relationships: is a type of regulation of localization [GO:0032879]; regulates synaptic vesicle clustering [GO:0097091] References: PMID:21513708 Subtypes: negative regulation of synaptic vesicle clustering [GO:2000808], positive regulation of synaptic vesicle clustering [GO:2000809] Definition: Any process that modulates the frequency, rate or extent of synaptic vesicle clustering.